contractile ring contraction [GO:0036213] (biological process) Note: This term can be used to annotate contraction of either bacterial or fungal contractile rings. Definition: The process of an actomyosin ring getting smaller in diameter. Sources: GOC:mah, GOC:vw Also known as: contractile ring constriction Subtypes: actomyosin contractile ring contraction [GO:0000916] Relationships: is a type of cytokinetic process [GO:0032506]; is part of GO:0061640